{
  "term_id": "UNKNOWN:0003",
  "term_label": "Unknown cellular component",
  "gene_symbol": "NIBAN1",
  "gene": "UniProtKB:Q9BZQ8",
  "gene_name": "Protein Niban 1"
}